{
  "term_id": "GO:0006915",
  "gene_symbol": "CASP8",
  "gene_name": "Caspase-8",
  "gene": "UniProtKB:Q14790",
  "term_label": "apoptotic process"
}